{
  "term_id": "GO:0007399",
  "term_label": "nervous system development",
  "gene_name": "Macrophage-stimulating protein receptor",
  "gene_symbol": "MST1R",
  "gene": "UniProtKB:Q04912"
}